{
  "term_label": "nucleus",
  "term_id": "GO:0005634",
  "gene_symbol": "TFDP1",
  "gene_name": "Transcription factor Dp-1",
  "gene": "UniProtKB:Q14186"
}